{
  "gene_symbol": "SPRTN",
  "gene_name": "DNA-dependent metalloprotease SPRTN",
  "term_id": "GO:0031593",
  "gene": "UniProtKB:Q9H040",
  "term_label": "polyubiquitin modification-dependent protein binding"
}